{
  "gene_symbol": "GIPC1",
  "gene": "UniProtKB:O14908",
  "term_label": "Unknown biological process",
  "gene_name": "PDZ domain-containing protein GIPC1",
  "term_id": "UNKNOWN:0002"
}